metaphase/anaphase transition of mitotic cell cycle [GO:0007091] (biological process) References: PMID:10465783 Sources: GOC:mtg_cell_cycle Regulation: regulated by GO:0030071; negatively regulated by negative regulation of mitotic metaphase/anaphase transition [GO:0045841]; positively regulated by positive regulation of mitotic metaphase/anaphase transition [GO:0045842] Relationships: is a type of mitotic cell cycle phase transition [GO:0044772]; is a type of metaphase/anaphase transition of cell cycle [GO:0044784] Definition: The cell cycle process in which a cell progresses from metaphase to anaphase during mitosis, triggered by the activation of the anaphase promoting complex by Cdc20/Sleepy homolog which results in the degradation of Securin. Also known as: metaphase/anaphase transition by anaphase-promoting complex-dependent proteasomal ubiquitin-dependent protein catabolic process, mitotic metaphase/anaphase transition